{
  "gene": "UniProtKB:P54868",
  "gene_symbol": "HMGCS2",
  "term_label": "hydroxymethylglutaryl-CoA synthase activity",
  "gene_name": "Hydroxymethylglutaryl-CoA synthase, mitochondrial",
  "term_id": "GO:0004421"
}